positive regulation of dendrite development [GO:1900006] (biological process) Sources: GOC:TermGenie Definition: Any process that activates or increases the frequency, rate or extent of dendrite development. Also known as: up regulation of dendrite development Relationships: is a type of GO:0010976; is a type of regulation of dendrite development [GO:0050773]; is a type of positive regulation of developmental process [GO:0051094]; positively regulates GO:0016358